{
  "term_label": "histidine transport",
  "gene_symbol": "SLC38A3",
  "gene_name": "Sodium-coupled neutral amino acid transporter 3",
  "term_id": "GO:0015817",
  "gene": "UniProtKB:Q99624"
}